{
  "gene_name": "NEDD4-binding protein 3",
  "gene": "UniProtKB:O15049",
  "term_label": "Unknown biological process",
  "gene_symbol": "N4BP3",
  "term_id": "UNKNOWN:0002"
}